positive regulation of nigerotriose transport [GO:1900359] (biological process) Also known as: up regulation of nigerotriose transport, up-regulation of nigerotriose transport, upregulation of nigerotriose transport, activation of nigerotriose transport Sources: GOC:TermGenie, GOC:mengo_curators Relationships: is a type of positive regulation of transport [GO:0051050]; is a type of regulation of nigerotriose transport [GO:1900357]; positively regulates nigerotriose transport [GO:2001091] Definition: Any process that activates or increases the frequency, rate or extent of nigerotriose transport.